{
  "term_id": "GO:0004633",
  "gene_symbol": "PPCDC",
  "gene_name": "Phosphopantothenoylcysteine decarboxylase",
  "gene": "UniProtKB:Q96CD2",
  "term_label": "phosphopantothenoylcysteine decarboxylase activity"
}